peptide transmembrane transporter activity [GO:1904680] (molecular function) Relationships: is a type of transmembrane transporter activity [GO:0022857] Definition: Enables the transfer of a peptide from one side of a membrane to the other. Subtypes: GO:0015333, ABC-type peptide transporter activity [GO:0015440] Sources: GOC:TermGenie, GOC:vw, GO_REF:0000070 Also known as: peptide transporter activity, peptide uptake permease activity